{
  "term_label": "Unknown molecular function",
  "gene": "UniProtKB:Q6XE38",
  "term_id": "UNKNOWN:0001",
  "gene_name": "Secretoglobin family 1D member 4",
  "gene_symbol": "SCGB1D4"
}